{
  "gene_symbol": "WWC3",
  "gene_name": "Protein WWC3",
  "term_label": "cell migration",
  "term_id": "GO:0016477",
  "gene": "UniProtKB:Q9ULE0"
}